embryonic brain development [GO:1990403] (biological process) References: PMID:15918910 Relationships: is a type of embryonic organ development [GO:0048568] Definition: The process occurring during the embryonic phase whose specific outcome is the progression of the brain over time, from its formation to the mature structure.